{
  "gene": "UniProtKB:O00204",
  "term_id": "GO:0005737",
  "term_label": "cytoplasm",
  "gene_name": "Sulfotransferase 2B1",
  "gene_symbol": "SULT2B1"
}